{
  "gene_symbol": "ABR",
  "gene_name": "Active breakpoint cluster region-related protein",
  "term_label": "membrane",
  "gene": "UniProtKB:Q12979",
  "term_id": "GO:0016020"
}